{
  "term_label": "Unknown molecular function",
  "gene_name": "Peptidyl-prolyl cis-trans isomerase FKBP14",
  "gene_symbol": "FKBP14",
  "gene": "UniProtKB:Q9NWM8",
  "term_id": "UNKNOWN:0001"
}